{
  "gene_symbol": "CD40",
  "term_id": "GO:0035631",
  "gene": "UniProtKB:P25942",
  "gene_name": "Tumor necrosis factor receptor superfamily member 5",
  "term_label": "CD40 receptor complex"
}